{
  "gene_symbol": "OR51D1",
  "gene": "UniProtKB:Q8NGF3",
  "term_id": "UNKNOWN:0002",
  "gene_name": "Olfactory receptor 51D1",
  "term_label": "Unknown biological process"
}